{
  "gene_symbol": "GKN3P",
  "term_label": "Unknown molecular function",
  "gene": "UniProtKB:P0CG01",
  "gene_name": "Gastrokine-3",
  "term_id": "UNKNOWN:0001"
}